rRNA N-glycosylase activity [GO:0030598] (molecular function) Definition: Catalysis of the hydrolysis of the N-glycosylic bond at A-4324 in 28S rRNA from rat ribosomes or corresponding sites in 28S RNA from other species. Sources: EC:3.2.2.22, GOC:mah Also known as: rRNA N-glycosidase activity, RNA N-glycosidase activity, gelonin, mirabilis antiviral protein, momorcochin-S, nigrin b, rRNA N-glycohydrolase activity, ribosomal ribonucleate N-glycosidase activity, ricin, saporins Relationships: is a type of RNA glycosylase activity [GO:0030597]; is a type of catalytic activity, acting on a rRNA [GO:0140102]